{
  "term_id": "GO:0030182",
  "gene_symbol": "RTN3",
  "gene_name": "Reticulon-3",
  "gene": "UniProtKB:O95197",
  "term_label": "neuron differentiation"
}